{
  "term_id": "GO:0038202",
  "gene_name": "Ribosomal protein S6 kinase alpha-3",
  "gene": "UniProtKB:P51812",
  "gene_symbol": "RPS6KA3",
  "term_label": "TORC1 signaling"
}